{
  "term_id": "GO:0035249",
  "term_label": "synaptic transmission, glutamatergic",
  "gene": "UniProtKB:P42261",
  "gene_name": "Glutamate receptor 1",
  "gene_symbol": "GRIA1"
}